{
  "term_id": "GO:0043025",
  "term_label": "neuronal cell body",
  "gene": "UniProtKB:Q9BYH1",
  "gene_name": "Seizure 6-like protein",
  "gene_symbol": "SEZ6L"
}